{
  "gene": "UniProtKB:Q9H6I2",
  "term_id": "GO:0045944",
  "gene_symbol": "SOX17",
  "gene_name": "Transcription factor SOX-17",
  "term_label": "positive regulation of transcription by RNA polymerase II"
}